{
  "term_id": "GO:0005886",
  "term_label": "plasma membrane",
  "gene_name": "Stomatin",
  "gene_symbol": "STOM",
  "gene": "UniProtKB:P27105"
}